{
  "gene_name": "Midkine",
  "gene": "UniProtKB:P21741",
  "term_label": "Unknown cellular component",
  "gene_symbol": "MDK",
  "term_id": "UNKNOWN:0003"
}